ATP-dependent DNA damage sensor activity [GO:0140664] (molecular function) References: PMID:33302090, PMID:33510387 Definition: A molecule that recognises toxic DNA structures, and initiates a signaling response, driven by ATP hydrolysis. Also known as: ATP-dependent DNA damage sensing activity Relationships: is_a ATP-dependent activity, acting on DNA [GO:0008094]; is a type of DNA damage sensor activity [GO:0140612]